{
  "gene": "UniProtKB:Q9UMS4",
  "term_label": "mRNA splicing, via spliceosome",
  "term_id": "GO:0000398",
  "gene_symbol": "PRPF19",
  "gene_name": "Pre-mRNA-processing factor 19"
}